cAMP-dependent protein kinase regulator activity [GO:0008603] (molecular function) Subtypes: GO:0004862 Definition: Modulation of the activity of the enzyme cAMP-dependent protein kinase. Also known as: 3',5' cAMP-dependent protein kinase regulator activity, 3',5'-cAMP-dependent protein kinase regulator activity, adenosine 3',5'-cyclophosphate-dependent protein kinase regulator activity, cyclic AMP-dependent protein kinase regulator activity, cAMP-dependent protein kinase, intrinsic regulator activity Sources: GOC:ai Relationships: is_a GO:0019887; regulates cAMP-dependent protein kinase activity [GO:0004691]